{
  "term_label": "Unknown biological process",
  "term_id": "UNKNOWN:0002",
  "gene": "UniProtKB:A4D1Z8",
  "gene_name": "Grifin",
  "gene_symbol": "GRIFIN"
}